{
  "gene_name": "U3 small nucleolar RNA-associated protein 4 homolog",
  "gene_symbol": "UTP4",
  "term_label": "maturation of SSU-rRNA from tricistronic rRNA transcript (SSU-rRNA, 5.8S rRNA, LSU-rRNA)",
  "gene": "UniProtKB:Q969X6",
  "term_id": "GO:0000462"
}